{
  "term_id": "GO:0006954",
  "gene_symbol": "PF4",
  "gene_name": "Platelet factor 4",
  "term_label": "inflammatory response",
  "gene": "UniProtKB:P02776"
}